{
  "gene_name": "Cytokine-dependent hematopoietic cell linker",
  "gene": "UniProtKB:Q7Z7G1",
  "gene_symbol": "CLNK",
  "term_id": "GO:0030674",
  "term_label": "protein-macromolecule adaptor activity"
}